{
  "term_id": "GO:0030833",
  "gene_symbol": "HAX1",
  "term_label": "regulation of actin filament polymerization",
  "gene": "UniProtKB:O00165",
  "gene_name": "HCLS1-associated protein X-1"
}